{
  "gene_symbol": "CCR4",
  "gene": "UniProtKB:P51679",
  "term_label": "cell chemotaxis",
  "term_id": "GO:0060326",
  "gene_name": "C-C chemokine receptor type 4"
}